membrane [GO:0016020] (cellular component) Subtypes: GO:0005628, annulate lamellae [GO:0005642], GO:0005886, GO:0005905, outer membrane [GO:0019867], GO:0031090, phagophore assembly site membrane [GO:0034045], photosynthetic membrane [GO:0034357], ascus membrane [GO:0036362], nuclear outer membrane-endoplasmic reticulum membrane network [GO:0042175], coated membrane [GO:0048475], prospore membrane leading edge [GO:0070056], plasma membrane region [GO:0098590], membrane microdomain [GO:0098857], pathogen-containing vacuole membrane [GO:0140221], spore inner membrane [GO:0140549] Definition: A lipid bilayer along with all the proteins and protein complexes embedded in it and attached to it. Also known as: integral component of membrane, integral to membrane, membrane region, region of membrane, whole membrane, transmembrane Relationships: is a type of GO:0110165 Sources: GOC:dos, GOC:mah, ISBN:0815316194